{
  "term_id": "GO:0004568",
  "term_label": "chitinase activity",
  "gene": "UniProtKB:Q9BZP6",
  "gene_name": "Acidic mammalian chitinase",
  "gene_symbol": "CHIA"
}